mitochondrial ribosome binding [GO:0097177] (molecular function) Relationships: is a type of ribosome binding [GO:0043022] Subtypes: mitochondrial large ribosomal subunit binding [GO:0140978], mitochondrial small ribosomal subunit binding [GO:0180065] Definition: Binding to a mitochondrial ribosome. References: PMID:20739282 Sources: GOC:ans